{
  "gene_name": "GTPase HRas",
  "term_label": "Ras protein signal transduction",
  "gene_symbol": "HRAS",
  "term_id": "GO:0007265",
  "gene": "UniProtKB:P01112"
}